{
  "gene_name": "Cholesterol side-chain cleavage enzyme, mitochondrial",
  "gene_symbol": "CYP11A1",
  "term_label": "mitochondrial inner membrane",
  "gene": "UniProtKB:P05108",
  "term_id": "GO:0005743"
}